methylguanidinase activity [GO:0050098] (molecular function) Definition: Catalysis of the reaction: H2O + methylguanidine = methylammonium + urea. Sources: EC:3.5.3.16, RHEA:11764 Relationships: is a type of hydrolase activity, acting on carbon-nitrogen (but not peptide) bonds, in linear amidines [GO:0016813] Also known as: methylguanidine amidinohydrolase activity, methylguanidine hydrolase activity